regulation of cellular response to iron ion starvation [GO:1901966] (BP) Definition: Any process that modulates the frequency, rate or extent of cellular response to iron ion starvation. Subtypes: GO:1901967 References: PMID:23115244 Sources: GOC:TermGenie Relationships: is a type of regulation of response to nutrient levels [GO:0032107]; is a type of regulation of cellular response to stress [GO:0080135]; regulates cellular response to iron ion starvation [GO:0010106]